{
  "term_id": "GO:0050853",
  "gene_symbol": "LCK",
  "gene": "UniProtKB:P06239",
  "term_label": "B cell receptor signaling pathway",
  "gene_name": "Tyrosine-protein kinase Lck"
}